{
  "gene": "UniProtKB:P62314",
  "gene_name": "Small nuclear ribonucleoprotein Sm D1",
  "term_label": "RNA binding",
  "gene_symbol": "SNRPD1",
  "term_id": "GO:0003723"
}